male mating behavior [GO:0060179] (biological process) Subtypes: male courtship behavior [GO:0008049], response to hermaphrodite contact [GO:0034606], GO:0034607, GO:0034608, spicule insertion [GO:0034609] Definition: The specific behavior of a male organism that is associated with reproduction. Regulation: regulated by regulation of male mating behavior [GO:1902435]; negatively regulated by negative regulation of male mating behavior [GO:1902436]; positively regulated by positive regulation of male mating behavior [GO:1902437] Relationships: is_a mating behavior [GO:0007617] Sources: GOC:dph, GOC:pr, GOC:tb